CSL-Notch-Mastermind transcription factor complex [GO:1990433] (cellular component) Definition: A DNA-binding transcription factor complex consisting of CSL and mastermind proteins in complex with the cleaved, intracellular domain of Notch. It is required for both repression and activation of Notch target genes. Relationships: is a type of RNA polymerase II transcription regulator complex [GO:0090575] References: PMID:16530045 Sources: GOC:bhm, GOC:dos Also known as: CSL-NotchIC-MASTERMIND complex